ribonuclease M5 activity [GO:0043822] (MF) Relationships: is a type of RNA endonuclease activity producing 5'-phosphomonoesters, hydrolytic mechanism [GO:0016891] Also known as: 5S ribosomal RNA maturation endonuclease activity, 5S ribosomal maturation nuclease activity, RNase M5 activity Definition: Catalysis of the endonucleolytic cleavage of RNA, removing 21 and 42 nucleotides, respectively, from the 5'- and 3'-termini of a 5S-rRNA precursor. References: PMID:402365